infected host cell surface knob [GO:0020030] (cellular component) Sources: GOC:mb Definition: Protrusion that develops in the plasma membrane of a parasitized erythrocyte. An example of this component is found in Plasmodium species. Relationships: is a type of host cell cytoplasm part [GO:0033655]